positive regulation of gerfelin biosynthetic process [GO:1900688] (biological process) Definition: Any process that activates or increases the frequency, rate or extent of gerfelin biosynthetic process. Relationships: is a type of positive regulation of small molecule metabolic process [GO:0062013]; is a type of positive regulation of secondary metabolite biosynthetic process [GO:1900378]; is a type of regulation of gerfelin biosynthetic process [GO:1900686]; positively regulates gerfelin biosynthetic process [GO:1900578] Also known as: activation of gerfelin anabolism, activation of gerfelin biosynthesis, activation of gerfelin formation, activation of gerfelin synthesis, positive regulation of gerfelin anabolism, positive regulation of gerfelin biosynthesis, positive regulation of gerfelin formation, positive regulation of gerfelin synthesis, up regulation of gerfelin anabolism, up regulation of gerfelin biosynthesis, up regulation of gerfelin biosynthetic process, up regulation of gerfelin formation, up regulation of gerfelin synthesis, up-regulation of gerfelin anabolism, up-regulation of gerfelin biosynthesis, up-regulation of gerfelin biosynthetic process, up-regulation of gerfelin formation, up-regulation of gerfelin synthesis, upregulation of gerfelin anabolism, upregulation of gerfelin biosynthesis, upregulation of gerfelin biosynthetic process, upregulation of gerfelin formation, upregulation of gerfelin synthesis, activation of gerfelin biosynthetic process Sources: GOC:TermGenie, GOC:di